bis(5'-adenosyl)-hexaphosphatase activity [GO:0034431] (molecular function) References: PMID:10085096, PMID:9450008 Sources: RHEA:32047 Also known as: AP(6)A hydrolase activity, AP-6-A hydrolase activity, AP6A hydrolase activity, diadenosine 5',5'''-P1,P6-hexaphosphate hydrolase activity Relationships: is a type of GO:0016462 Definition: Catalysis of the reaction: P1-P6-bis(5'-adenosyl) hexaphosphate + H2O = AMP + adenosine 5'-pentaphosphate.